{
  "term_label": "chemical synaptic transmission",
  "gene_symbol": "CACNB3",
  "gene": "UniProtKB:P54284",
  "term_id": "GO:0007268",
  "gene_name": "Voltage-dependent L-type calcium channel subunit beta-3"
}